right posteriolateral basal body [GO:1902674] (cellular component) References: PMID:16607022, PMID:5961344 Sources: GOC:TermGenie, GOC:giardia, GO_REF:0000064, ISBN:9780124260207 Definition: Any ciliary basal body that is part of a right posteriolateral flagellum found in Giardia species (trophozoite stage). Relationships: is a type of GO:0036064; is part of right posteriolateral flagellum [GO:0097557] Note: Note that we deem cilium and microtubule-based flagellum to be equivalent. Also note that, due to the asymmetric nature of the Giardia trophozoite, this term is defined spatially as the trophozoite is viewed from the dorsal side, with the two nuclei dorsal to the ventral disc, and the ventral disc toward the anterior. Also known as: cilial basal body of right posteriolateral cilium, cilial basal body of right posteriolateral flagellum, cilial basal body of right posterolateral cilium, cilial basal body of right posterolateral flagellum, ciliary basal body of right posteriolateral cilium, ciliary basal body of right posteriolateral flagellum, ciliary basal body of right posterolateral cilium, ciliary basal body of right posterolateral flagellum, cilium basal body of right posteriolateral cilium, cilium basal body of right posteriolateral flagellum, cilium basal body of right posterolateral cilium, cilium basal body of right posterolateral flagellum, microtubule basal body of right posteriolateral cilium, microtubule basal body of right posteriolateral flagellum, microtubule basal body of right posterolateral cilium, microtubule basal body of right posterolateral flagellum, right posteriolateral flagellum ciliary basal body